{
  "term_label": "regulation of transcription by RNA polymerase II",
  "term_id": "GO:0006357",
  "gene_name": "TNFAIP3-interacting protein 3",
  "gene": "UniProtKB:Q96KP6",
  "gene_symbol": "TNIP3"
}